riboflavin transport [GO:0032218] (biological process) References: PMID:16204239 Sources: GOC:rn Definition: The directed movement of riboflavin into, out of or within a cell, or between cells, by means of some agent such as a transporter or pore. Riboflavin (vitamin B2) is a water-soluble B-complex vitamin, converted in the cell to FMN and FAD, cofactors required for the function of flavoproteins. Relationships: is a type of GO:0015711; is_a vitamin transport [GO:0051180]; is a type of nitrogen compound transport [GO:0071705]